{
  "gene": "UniProtKB:P10747",
  "term_label": "Unknown molecular function",
  "term_id": "UNKNOWN:0001",
  "gene_name": "T-cell-specific surface glycoprotein CD28",
  "gene_symbol": "CD28"
}